{
  "term_id": "UNKNOWN:0001",
  "gene_name": "Protein FAM163A",
  "gene_symbol": "FAM163A",
  "gene": "UniProtKB:Q96GL9",
  "term_label": "Unknown molecular function"
}